{
  "term_label": "nucleus",
  "term_id": "GO:0005634",
  "gene": "UniProtKB:Q32MQ0",
  "gene_name": "Zinc finger protein 750",
  "gene_symbol": "ZNF750"
}